thyroid-stimulating hormone signaling pathway [GO:0038194] (biological process) Relationships: is a type of G protein-coupled receptor signaling pathway [GO:0007186] References: PMID:10809230 Sources: GOC:gap Definition: A G protein-coupled receptor signaling pathway initiated by thyroid-stimulating hormone (thyrotropin) binding to its receptor on the surface of a target cell, and ending with the regulation of a downstream cellular process, e.g. transcription. Also known as: TSH signaling pathway, thyrotropin signaling pathway